{
  "term_id": "UNKNOWN:0001",
  "gene_symbol": "CIMAP1C",
  "gene_name": "Outer dense fiber protein 3-like protein 1",
  "gene": "UniProtKB:Q8IXM7",
  "term_label": "Unknown molecular function"
}